{
  "gene_symbol": "SPTBN1",
  "term_id": "GO:0030036",
  "gene_name": "Spectrin beta chain, non-erythrocytic 1",
  "term_label": "actin cytoskeleton organization",
  "gene": "UniProtKB:Q01082"
}